{
  "gene": "UniProtKB:P29322",
  "gene_name": "Ephrin type-A receptor 8",
  "term_id": "GO:0007411",
  "term_label": "axon guidance",
  "gene_symbol": "EPHA8"
}